{
  "term_id": "GO:0030335",
  "gene": "UniProtKB:Q92854",
  "term_label": "positive regulation of cell migration",
  "gene_symbol": "SEMA4D",
  "gene_name": "Semaphorin-4D"
}